extrinsic component of postsynaptic density membrane [GO:0099147] (cellular component) Definition: The component of the postsynaptic density membrane consisting of gene products and protein complexes that are loosely bound to one of its surfaces, but not integrated into the hydrophobic region. Relationships: is a type of extrinsic component of postsynaptic specialization membrane [GO:0098892]; is part of GO:0098839 Sources: GOC:autophagy, GOC:mf